{
  "gene_name": "Zinc finger protein GLI2",
  "term_id": "GO:0006357",
  "term_label": "regulation of transcription by RNA polymerase II",
  "gene": "UniProtKB:P10070",
  "gene_symbol": "GLI2"
}